visceral peritoneum development [GO:1904818] (biological process) References: PMID:15840053 Sources: GOC:TermGenie, GOC:dph, GO_REF:0000094 Relationships: is a type of anatomical structure development [GO:0048856]; is part of peritoneum development [GO:1904820] Definition: The process whose specific outcome is the progression of a visceral peritoneum over time, from its formation to the mature structure.